{
  "gene_symbol": "PLEC",
  "term_label": "ankyrin binding",
  "gene_name": "Plectin",
  "term_id": "GO:0030506",
  "gene": "UniProtKB:Q15149"
}